{
  "gene_symbol": "NCEH1",
  "gene": "UniProtKB:Q6PIU2",
  "gene_name": "Neutral cholesterol ester hydrolase 1",
  "term_label": "Unknown cellular component",
  "term_id": "UNKNOWN:0003"
}